{
  "term_label": "protein-glucosylgalactosylhydroxylysine glucosidase activity",
  "gene": "UniProtKB:Q32M88",
  "gene_name": "Protein-glucosylgalactosylhydroxylysine glucosidase",
  "gene_symbol": "PGGHG",
  "term_id": "GO:0047402"
}